{
  "gene_name": "Peroxisome proliferator-activated receptor gamma",
  "term_label": "negative regulation of cholesterol storage",
  "gene": "UniProtKB:P37231",
  "gene_symbol": "PPARG",
  "term_id": "GO:0010887"
}